acyltransferase activity, transferring groups other than amino-acyl groups [GO:0016747] (molecular function) Sources: EC:2.3.1.- Also known as: transferase activity, transferring acyl groups other than amino-acyl groups, transferase activity, transferring groups other than amino-acyl groups Definition: Catalysis of the transfer of an acyl group, other than amino-acyl, from one compound (donor) to another (acceptor). Relationships: is a type of acyltransferase activity [GO:0016746] Subtypes: fatty acid synthase activity [GO:0004312], 3-oxoacyl-[acyl-carrier-protein] synthase activity [GO:0004315], GO:0008374, 8-amino-7-oxononanoate synthase activity [GO:0008710], Kdo2-lipid IVA acyltransferase activity [GO:0008913], GO:0008951, fatty acid elongase activity [GO:0009922], naringenin-chalcone synthase activity [GO:0016210], GO:0016407, GO:0016408, palmitoyltransferase activity [GO:0016409], N-acyltransferase activity [GO:0016410], S-acyltransferase activity [GO:0016417], malonyltransferase activity [GO:0016420], succinyltransferase activity [GO:0016748], GO:0016752, lipoyltransferase activity [GO:0017118], benzoyl acetate-CoA thiolase activity [GO:0018711], 3-hydroxybutyryl-CoA thiolase activity [GO:0018712], GO:0018713, myristoyltransferase activity [GO:0019107], 6'-deoxychalcone synthase activity [GO:0033808], anthocyanin 6''-O-malonyltransferase activity [GO:0033809], anthocyanin 5-O-glucoside 6'''-O-malonyltransferase activity [GO:0033810], flavonol-3-O-triglucoside O-coumaroyltransferase activity [GO:0033811], biphenyl synthase activity [GO:0033815], beta-ketoacyl-acyl-carrier-protein synthase III activity [GO:0033818], lipoyl(octanoyl) transferase activity [GO:0033819], mycothiol synthase activity [GO:0035447], (R)-citramalate synthase activity [GO:0043714], 3-keto-5-aminohexanoate cleavage activity [GO:0043720], dihydrolipoamide branched chain acyltransferase activity [GO:0043754], GO:0043772, phosphate:acyl-[acyl carrier protein] acyltransferase activity [GO:0043811], GO:0043875, CO-methylating acetyl-CoA synthase activity [GO:0043884], GO:0046027, pyruvyltransferase activity [GO:0046919], GO:0047168, GO:0047176, glycerophospholipid arachidonoyl-transferase (CoA-independent) activity [GO:0047177], glycerophospholipid acyltransferase (CoA-dependent) activity [GO:0047178], tetrahydroxybenzophenone synthase activity [GO:0047181], alcohol O-cinnamoyltransferase activity [GO:0047182], anthocyanin 5-(6'''-hydroxycinnamoyltransferase) activity [GO:0047183], 2,3-diaminopropionate N-oxalyltransferase activity [GO:0047189], GO:0047201, 13-hydroxylupinine O-tigloyltransferase activity [GO:0047203], agmatine N4-coumaroyltransferase activity [GO:0047634], GO:0047672, erythronolide synthase activity [GO:0047879], glutamine N-phenylacetyltransferase activity [GO:0047947], glycine N-benzoyltransferase activity [GO:0047962], glycine N-choloyltransferase activity [GO:0047963], mycocerosate synthase activity [GO:0050111], ornithine N-benzoyltransferase activity [GO:0050156], GO:0050182, pinosylvin synthase activity [GO:0050198], piperidine N-piperoyltransferase activity [GO:0050199], rosmarinate synthase activity [GO:0050266], trehalose O-mycolyltransferase activity [GO:0050348], trihydroxystilbene synthase activity [GO:0050350], tyramine N-feruloyltransferase activity [GO:0050366], propionyl-CoA C2-trimethyltridecanoyltransferase activity [GO:0050632], GO:0050634, GO:0050635, vinorine synthase activity [GO:0050636], lovastatin nonaketide synthase activity [GO:0050637], GO:0050641, 2-alpha-hydroxytaxane 2-O-benzoyltransferase activity [GO:0050642], hydroxycinnamoyltransferase activity [GO:0050734], peptide alpha-N-propionyltransferase activity [GO:0061607], GO:0061711, beta-ketodecanoyl-[acyl-carrier-protein] synthase activity [GO:0061990], lysophospholipid acyltransferase activity [GO:0071617], GO:0090430, GO:0090439, GO:0102080, demethoxycurcumin synthase activity [GO:0102103], curcumin synthase activity [GO:0102106], (Z)-3-hexen-1-ol acetyltransferase activity [GO:0102165], omega-hydroxypalmitate O-sinapoyl transferase activity [GO:0102406], bisdemethoxycurcumin synthase activity [GO:0102452], GO:0102453, cyanidin 3-O-[2''-O-(xylosyl)-6''-O-(p-coumaroyl) glucoside] 5-O-glucoside malonyltransferase activity [GO:0102585], acetyl-coenzyme A:acetyl alcohol acetyltransferase activity [GO:0102720], trihydroxybenzophenone synthase activity [GO:0102735], GO:0102801, GO:0102922, GO:0102923, GO:0102971, GO:0102973, GO:0103118, glycero-3-phosphocholine acyltransferase activity [GO:0106158], GO:0106341, NAD-dependent protein lipoamidase activity [GO:0106419], NAD-dependent protein biotinidase activity [GO:0106420], NAD-dependent protein demyristoylase activity [GO:0140773], NAD-dependent protein depalmitoylase activity [GO:0140774], NAD-dependent protein lysine deacylase activity [GO:0141218], NAD-dependent protein decrotonylase activity [GO:0160011], NAD-dependent protein de-2-hydroxyisobutyrylase activity [GO:0160013], bis(monoacylglycero)phosphate synthase activity [GO:0160121], palmitoleoyltransferase activity [GO:1990698]